{
  "term_id": "GO:0006357",
  "gene": "UniProtKB:Q8TDQ0",
  "gene_name": "Hepatitis A virus cellular receptor 2",
  "term_label": "regulation of transcription by RNA polymerase II",
  "gene_symbol": "HAVCR2"
}